positive regulation of receptor signaling pathway via JAK-STAT [GO:0046427] (biological process) Relationships: is a type of regulation of receptor signaling pathway via JAK-STAT [GO:0046425]; is a type of positive regulation of receptor signaling pathway via STAT [GO:1904894]; positively regulates cell surface receptor signaling pathway via JAK-STAT [GO:0007259] Sources: GOC:bf Definition: Any process that activates or increases the frequency, rate or extent of the JAK-STAT signaling pathway activity. Also known as: up regulation of JAK-STAT cascade, up-regulation of JAK-STAT cascade, upregulation of JAK-STAT cascade, activation of JAK-STAT cascade, positive regulation of STAT protein import into nucleus, positive regulation of STAT protein nuclear translocation, stimulation of JAK-STAT cascade